{
  "gene_symbol": "EXOSC7",
  "gene": "UniProtKB:Q15024",
  "gene_name": "Exosome complex component RRP42",
  "term_id": "GO:0034476",
  "term_label": "U5 snRNA 3'-end processing"
}